{
  "term_id": "GO:0005739",
  "gene_name": "Succinate dehydrogenase assembly factor 2, mitochondrial",
  "term_label": "mitochondrion",
  "gene": "UniProtKB:Q9NX18",
  "gene_symbol": "SDHAF2"
}